histone H4 demethylase activity [GO:0141058] (molecular function) Definition: Catalysis of the removal of a methyl group from a modified lysine residue of the histone H4 protein. This is a dioxygenase reaction that is dependent on Fe(II) and 2-oxoglutarate. References: PMID:17947579 Relationships: is a type of GO:0032452 Subtypes: histone H4R3 demethylase activity [GO:0033749], histone H4K20 demethylase activity [GO:0035575]